{
  "gene": "UniProtKB:P11487",
  "term_id": "GO:0030334",
  "gene_symbol": "FGF3",
  "gene_name": "Fibroblast growth factor 3",
  "term_label": "regulation of cell migration"
}